{
  "term_label": "transcription regulator complex",
  "gene_name": "Retinoblastoma-like protein 1",
  "gene": "UniProtKB:P28749",
  "term_id": "GO:0005667",
  "gene_symbol": "RBL1"
}